{
  "gene_symbol": "RNF135",
  "gene": "UniProtKB:Q8IUD6",
  "term_id": "GO:0005737",
  "term_label": "cytoplasm",
  "gene_name": "E3 ubiquitin-protein ligase RNF135"
}